{
  "gene": "UniProtKB:Q12800",
  "gene_symbol": "TFCP2",
  "term_label": "positive regulation of transcription by RNA polymerase II",
  "term_id": "GO:0045944",
  "gene_name": "Alpha-globin transcription factor CP2"
}